mitochondrial 2-oxoadipate transmembrane transport [GO:1990551] (biological process) Definition: The process in which 2-oxoadipate is transported across a mitochondrial membrane, into or out of the mitochondrion. References: PMID:11013234 Relationships: is a type of dicarboxylic acid transport [GO:0006835]; is a type of carboxylic acid transmembrane transport [GO:1905039]